methenyltetrahydrofolate cyclohydrolase activity [GO:0004477] (MF) Sources: EC:3.5.4.9 Also known as: 5,10-methenyl-THF cyclohydrolase activity, 5,10-methenyltetrahydrofolate 5-hydrolase (decyclizing), citrovorum factor cyclodehydrase activity, formyl-methenyl-methylenetetrahydrofolate synthetase (combined) Relationships: is_a cyclohydrolase activity [GO:0019238] Definition: Catalysis of the reaction: 5,10-methenyltetrahydrofolate + H2O = 10-formyltetrahydrofolate.